{
  "gene_symbol": "ERGIC1",
  "term_id": "GO:0005783",
  "gene_name": "Endoplasmic reticulum-Golgi intermediate compartment protein 1",
  "term_label": "endoplasmic reticulum",
  "gene": "UniProtKB:Q969X5"
}